diterpene phytoalexin precursor biosynthetic process [GO:0051504] (biological process) Also known as: diterpene phytoalexin precursor anabolism pathway, diterpene phytoalexin precursor formation pathway, diterpene phytoalexin precursor synthesis pathway Sources: MetaCyc:PWY-2981 Relationships: is_a GO:0046246; is part of GO:0051502 Definition: A branched pathway that produces the precursors to four structurally distinct types of polycyclic diterpenes. The pathway starts with the cyclization of geranylgeranyl diphosphate into ent-copalyl diphosphate and syn-copalyl diphosphate. The catalytic conversion by diterpene cyclases of these two compounds produces the four diterpene hydrocarbons which are precursors to the four structurally distinct classes of diterpene phytoalexins.